{
  "term_label": "negative regulation of glycogen biosynthetic process",
  "gene": "UniProtKB:Q9BT40",
  "gene_name": "Inositol polyphosphate 5-phosphatase K",
  "term_id": "GO:0045719",
  "gene_symbol": "INPP5K"
}